receptor tyrosine kinase binding [GO:0030971] (molecular function) Definition: Binding to a receptor that possesses protein tyrosine kinase activity. Sources: GOC:mah Also known as: transmembrane receptor protein tyrosine kinase ligand binding Relationships: is a type of GO:0005102; is a type of protein tyrosine kinase binding [GO:1990782] Subtypes: transmembrane receptor protein tyrosine kinase adaptor activity [GO:0005068]